negative regulation of microtubule depolymerization [GO:0007026] (BP) Sources: GOC:mah, ISBN:0815316194 Relationships: is_a negative regulation of microtubule polymerization or depolymerization [GO:0031111]; is a type of regulation of microtubule depolymerization [GO:0031114]; is a type of negative regulation of protein depolymerization [GO:1901880]; is a type of negative regulation of supramolecular fiber organization [GO:1902904]; negatively regulates microtubule depolymerization [GO:0007019] Also known as: down regulation of microtubule depolymerization, down-regulation of microtubule depolymerization, downregulation of microtubule depolymerization, microtubule stabilization, negative regulation of microtubule disassembly, inhibition of microtubule depolymerization, microtubule rescue, negative regulation of microtubule catastrophe Definition: Any process that stops, prevents, or reduces the frequency, rate or extent of microtubule depolymerization; prevention of depolymerization of a microtubule can result from binding by 'capping' at the plus end (e.g. by interaction with another cellular protein of structure) or by exposing microtubules to a stabilizing drug such as taxol. Subtypes: negative regulation of axonemal microtubule depolymerization [GO:0007027], negative regulation of astral microtubule depolymerization [GO:0032932]